{
  "gene_name": "Interleukin-11",
  "gene": "UniProtKB:P20809",
  "term_id": "GO:0005737",
  "term_label": "cytoplasm",
  "gene_symbol": "IL11"
}